{
  "term_id": "GO:0005085",
  "term_label": "guanyl-nucleotide exchange factor activity",
  "gene_name": "Elongation factor 1-delta",
  "gene": "UniProtKB:P29692",
  "gene_symbol": "EEF1D"
}